Nebenkern assembly [GO:0007287] (BP) Note: See also the cellular component term 'Nebenkern ; GO:0016006', and the fly_anatomy.ontology term 'Nebenkern ; FBbt:00004943'. Definition: Fusion of mitochondria during insect spermatid differentiation to form two masses, which wrap around each other to form a densely packed sphere called the Nebenkern. Also known as: Nebenkern formation References: PMID:9550716 Sources: GOC:bf, ISBN:0879694238 Relationships: is a type of developmental process involved in reproduction [GO:0003006]; is a type of organelle assembly [GO:0070925]; is part of spermatid development [GO:0007286]